{
  "term_id": "GO:0098978",
  "gene_symbol": "SRGAP2C",
  "gene": "UniProtKB:P0DJJ0",
  "term_label": "glutamatergic synapse",
  "gene_name": "SLIT-ROBO Rho GTPase-activating protein 2C"
}